{
  "gene": "UniProtKB:P26038",
  "gene_symbol": "MSN",
  "term_label": "positive regulation of protein localization to early endosome",
  "gene_name": "Moesin",
  "term_id": "GO:1902966"
}